{
  "term_label": "Unknown cellular component",
  "gene_name": "Coiled-coil domain-containing protein 32",
  "gene": "UniProtKB:Q9BV29",
  "term_id": "UNKNOWN:0003",
  "gene_symbol": "CCDC32"
}